trichoblast differentiation [GO:0010054] (biological process) Sources: GOC:tb Relationships: is a type of GO:0010053 Also known as: trichoblast cell differentiation Definition: The process in which a relatively unspecialized cell acquires the specialized features of a trichoblast, a root epidermal cell that will give rise to a root hair.